{
  "gene_name": "Kinesin-like protein KIF6",
  "gene": "UniProtKB:Q6ZMV9",
  "gene_symbol": "KIF6",
  "term_id": "GO:0005871",
  "term_label": "kinesin complex"
}